{
  "gene": "UniProtKB:Q7Z6J4",
  "term_id": "GO:0046847",
  "gene_name": "FYVE, RhoGEF and PH domain-containing protein 2",
  "gene_symbol": "FGD2",
  "term_label": "filopodium assembly"
}